{
  "term_label": "Unknown molecular function",
  "gene": "UniProtKB:Q02833",
  "gene_symbol": "RASSF7",
  "term_id": "UNKNOWN:0001",
  "gene_name": "Ras association domain-containing protein 7"
}